protein localization to ciliary inversin compartment [GO:1904108] (BP) Definition: A process in which a protein is transported to, or maintained in, a location within a ciliary inversin compartment. References: PMID:25335890 Sources: GOC:TermGenie, GOC:kmv, GO_REF:0000087 Relationships: is a type of protein localization to cilium [GO:0061512] Also known as: protein localisation in ciliary inversin compartment, protein localisation to ciliary inversin compartment, protein localization in ciliary inversin compartment